protein aggregate center assembly [GO:0140454] (BP) References: PMID:32075773 Also known as: PAC assembly, protein aggregate center formation, protein aggregate centre assembly Definition: The reversible aggregation of misfolded proteins and chaperones, formed to shield thermosensitive proteins from degradation until conditions allow disaggregation and refolding. Relationships: is a type of cellular component assembly [GO:0022607]